{
  "term_label": "cytokine-mediated signaling pathway",
  "gene_symbol": "LIFR",
  "term_id": "GO:0019221",
  "gene_name": "Leukemia inhibitory factor receptor",
  "gene": "UniProtKB:P42702"
}